B cell selection [GO:0002339] (BP) Subtypes: GO:0002340, peripheral B cell selection [GO:0002343], GO:0002346, GO:0002352 Relationships: is a type of immune system process [GO:0002376]; is part of GO:0030183 Also known as: B lymphocyte selection, B-cell selection, B-lymphocyte selection Sources: GOC:jal Definition: The process dependent upon B cell antigen receptor signaling in response to self or foreign antigen through which B cells are selected for survival.